{
  "gene_symbol": "XCR1",
  "term_id": "GO:0019722",
  "term_label": "calcium-mediated signaling",
  "gene": "UniProtKB:P46094",
  "gene_name": "Chemokine XC receptor 1"
}